{
  "term_label": "fast-twitch skeletal muscle fiber contraction",
  "gene": "UniProtKB:O15061",
  "term_id": "GO:0031443",
  "gene_symbol": "SYNM",
  "gene_name": "Synemin"
}